{
  "term_id": "GO:0008277",
  "term_label": "regulation of G protein-coupled receptor signaling pathway",
  "gene": "UniProtKB:Q8TEY7",
  "gene_symbol": "USP33",
  "gene_name": "Ubiquitin carboxyl-terminal hydrolase 33"
}